{
  "term_label": "phosphatidylinositol phosphate binding",
  "gene": "UniProtKB:Q8IV53",
  "term_id": "GO:1901981",
  "gene_symbol": "DENND1C",
  "gene_name": "DENN domain-containing protein 1C"
}